{
  "gene_symbol": "LMAN2",
  "term_id": "GO:0006888",
  "gene": "UniProtKB:Q12907",
  "gene_name": "Vesicular integral-membrane protein VIP36",
  "term_label": "endoplasmic reticulum to Golgi vesicle-mediated transport"
}